DnaB-DnaC-DnaT-PriA-PriB complex [GO:1990158] (cellular component) Also known as: DnaB-DnaC-DnaT-PriA-PriB preprimosome, phi-X174-type preprimosome References: PMID:8663105 Sources: GOC:bhm Definition: A protein-DNA complex consisting of the helicase loading complex DnaB-DnaC, replication restart proteins DnaT, PriA and PriB, and associated DNA. Involved in the restart of DNA replication after a stalled replication fork has been repaired. Relationships: is a type of pre-primosome complex [GO:1990099]; has part DnaB-DnaC complex [GO:1990100]